thrombopoietin receptor activity [GO:0038164] (molecular function) Definition: Combining with the glycoprotein thrombopoietin and transmitting the signal from one side of the membrane to the other to initiate a change in cell activity. Relationships: is_a GO:0004896; is part of thrombopoietin-mediated signaling pathway [GO:0038163] References: PMID:19630807 Sources: GOC:bf, GOC:signaling